{
  "gene_name": "Alpha-1,3-galactosyltransferase 2",
  "term_label": "glycosphingolipid biosynthetic process",
  "term_id": "GO:0006688",
  "gene_symbol": "A3GALT2",
  "gene": "UniProtKB:U3KPV4"
}